lactose synthase activity [GO:0004461] (molecular function) Also known as: UDP-galactose-glucose galactosyltransferase activity, UDP-galactose:D-glucose 4-beta-D-galactotransferase activity, UDPgalactose-glucose galactosyltransferase activity, UDPgalactose:D-glucose 4-beta-D-galactotransferase activity, lactose synthetase activity, uridine diphosphogalactose-glucose galactosyltransferase activity Definition: Catalysis of the reaction: UDP-galactose + D-glucose = UDP + lactose. Sources: EC:2.4.1.22 Relationships: is_a UDP-galactosyltransferase activity [GO:0035250]